organic acid metabolic process [GO:0006082] (biological process) Also known as: organic acid metabolism Subtypes: organic acid biosynthetic process [GO:0016053], organic acid catabolic process [GO:0016054], thiocyanate metabolic process [GO:0018969], naphthalenesulfonate metabolic process [GO:0018984], alkanesulfonate metabolic process [GO:0019694], organic acid phosphorylation [GO:0031388], oxoacid metabolic process [GO:0043436] Definition: The chemical reactions and pathways involving organic acids, any acidic compound containing carbon in covalent linkage. Sources: ISBN:0198506732 Relationships: is a type of GO:0044281